{
  "gene": "UniProtKB:Q15915",
  "gene_name": "Zinc finger protein ZIC 1",
  "gene_symbol": "ZIC1",
  "term_id": "GO:0000978",
  "term_label": "RNA polymerase II cis-regulatory region sequence-specific DNA binding"
}